{
  "gene_symbol": "OR9G4",
  "term_id": "GO:0007186",
  "term_label": "G protein-coupled receptor signaling pathway",
  "gene": "UniProtKB:Q8NGQ1",
  "gene_name": "Olfactory receptor 9G4"
}